{
  "term_label": "motile cilium",
  "gene": "UniProtKB:Q5T0N1",
  "gene_symbol": "CFAP70",
  "gene_name": "Cilia- and flagella-associated protein 70",
  "term_id": "GO:0031514"
}